{
  "term_id": "GO:0015189",
  "gene": "UniProtKB:Q6ZP29",
  "gene_name": "Lysosomal amino acid transporter 1 homolog",
  "term_label": "L-lysine transmembrane transporter activity",
  "gene_symbol": "SLC66A1"
}